{
  "gene": "UniProtKB:Q9HCR9",
  "gene_name": "Dual 3',5'-cyclic-AMP and -GMP phosphodiesterase 11A",
  "term_id": "GO:0004118",
  "gene_symbol": "PDE11A",
  "term_label": "3',5'-cGMP-stimulated cyclic-nucleotide phosphodiesterase activity"
}